{
  "gene": "UniProtKB:Q92934",
  "gene_symbol": "BAD",
  "term_id": "GO:0097191",
  "term_label": "extrinsic apoptotic signaling pathway",
  "gene_name": "Bcl2-associated agonist of cell death"
}